{
  "term_id": "GO:0032281",
  "term_label": "AMPA glutamate receptor complex",
  "gene": "UniProtKB:B8ZZ34",
  "gene_name": "Protein shisa-8",
  "gene_symbol": "SHISA8"
}